{
  "gene_name": "RANBP2-like and GRIP domain-containing protein 1",
  "term_id": "GO:0051168",
  "gene_symbol": "RGPD1",
  "term_label": "nuclear export",
  "gene": "UniProtKB:P0DJD0"
}